{
  "gene": "UniProtKB:Q99490",
  "gene_symbol": "AGAP2",
  "term_id": "GO:0043524",
  "term_label": "negative regulation of neuron apoptotic process",
  "gene_name": "Arf-GAP with GTPase, ANK repeat and PH domain-containing protein 2"
}